{
  "term_id": "UNKNOWN:0003",
  "gene_name": "T cell receptor beta joining 2-4",
  "gene": "UniProtKB:A0A0A0MT87",
  "term_label": "Unknown cellular component",
  "gene_symbol": "TRBJ2-4"
}